{
  "gene_symbol": "IL21",
  "term_label": "Unknown molecular function",
  "gene": "UniProtKB:Q9HBE4",
  "term_id": "UNKNOWN:0001",
  "gene_name": "Interleukin-21"
}